{
  "gene": "UniProtKB:O95810",
  "term_id": "GO:0005080",
  "gene_name": "Caveolae-associated protein 2",
  "term_label": "protein kinase C binding",
  "gene_symbol": "CAVIN2"
}